{
  "term_label": "NuA4 histone acetyltransferase complex",
  "gene": "UniProtKB:Q6S8J3",
  "gene_symbol": "POTEE",
  "term_id": "GO:0035267",
  "gene_name": "POTE ankyrin domain family member E"
}